{
  "gene_name": "Transmembrane protein 199",
  "gene_symbol": "TMEM199",
  "term_label": "endomembrane system",
  "gene": "UniProtKB:Q8N511",
  "term_id": "GO:0012505"
}